{
  "gene_symbol": "IL36A",
  "gene": "UniProtKB:Q9UHA7",
  "gene_name": "Interleukin-36 alpha",
  "term_id": "GO:0071222",
  "term_label": "cellular response to lipopolysaccharide"
}